dihydrobunolol dehydrogenase activity [GO:0047855] (molecular function) Sources: EC:1.1.1.160, RHEA:15925 Also known as: (+-)-5-[(tert-butylamino)-2'-hydroxypropoxy]-1,2,3,4-tetrahydro-1-naphthol:NADP+ oxidoreductase activity, bunolol reductase activity Definition: Catalysis of the reaction: dihydrobunolol + NADP+ = bunolol + H+ + NADPH. Relationships: is a type of oxidoreductase activity, acting on the CH-OH group of donors, NAD or NADP as acceptor [GO:0016616]